{
  "gene_symbol": "DACH2",
  "term_label": "regulation of transcription by RNA polymerase II",
  "gene": "UniProtKB:Q96NX9",
  "gene_name": "Dachshund homolog 2",
  "term_id": "GO:0006357"
}